sebaceous gland placode formation [GO:0060791] (biological process) Relationships: is a type of ectodermal placode formation [GO:0060788]; is part of GO:0048733 Definition: The developmental process in which a sebaceous gland placode forms. A sebaceous gland placode is a thickening of the ectoderm that will give rise to the sebaceous gland bud. Sources: GOC:dph, GOC:sdb_2009, GOC:tb